orlandin catabolic process [GO:1900820] (biological process) Also known as: orlandin breakdown, orlandin catabolism, orlandin degradation Sources: GOC:TermGenie, GOC:di Relationships: is_a secondary metabolite catabolic process [GO:0090487]; is a type of orlandin metabolic process [GO:1900819] Definition: The chemical reactions and pathways resulting in the breakdown of orlandin.